lactate catabolic process [GO:1903457] (biological process) Subtypes: aerobic lactate catabolic process [GO:1990484], anaerobic lactate catabolic process [GO:1990485] References: PMID:8941775 Sources: GOC:TermGenie, GOC:mengo_curators, GO_REF:0000068 Relationships: is a type of GO:0006089; is a type of monocarboxylic acid catabolic process [GO:0072329] Definition: The chemical reactions and pathways resulting in the breakdown of lactate. Also known as: lactate breakdown, lactate catabolism, lactate degradation